{
  "term_label": "chromatin",
  "gene_symbol": "MEN1",
  "gene_name": "Menin",
  "term_id": "GO:0000785",
  "gene": "UniProtKB:O00255"
}